{
  "gene_name": "EGF-containing fibulin-like extracellular matrix protein 2",
  "term_id": "GO:0005615",
  "term_label": "extracellular space",
  "gene": "UniProtKB:O95967",
  "gene_symbol": "EFEMP2"
}